{
  "term_id": "GO:0045197",
  "gene_name": "Microtubule cross-linking factor 1",
  "gene": "UniProtKB:Q9Y4B5",
  "gene_symbol": "MTCL1",
  "term_label": "establishment or maintenance of epithelial cell apical/basal polarity"
}